{
  "gene": "UniProtKB:Q9Y6I4",
  "term_id": "GO:0005634",
  "gene_symbol": "USP3",
  "gene_name": "Ubiquitin carboxyl-terminal hydrolase 3",
  "term_label": "nucleus"
}